{
  "gene": "UniProtKB:Q5T751",
  "term_id": "UNKNOWN:0001",
  "term_label": "Unknown molecular function",
  "gene_symbol": "LCE1C",
  "gene_name": "Late cornified envelope protein 1C"
}